{
  "term_id": "GO:0045109",
  "gene_name": "Keratin, type I cytoskeletal 13",
  "gene_symbol": "KRT13",
  "gene": "UniProtKB:P13646",
  "term_label": "intermediate filament organization"
}